{
  "gene_name": "Homeobox protein SIX2",
  "term_id": "GO:0005667",
  "term_label": "transcription regulator complex",
  "gene_symbol": "SIX2",
  "gene": "UniProtKB:Q9NPC8"
}